{
  "gene": "UniProtKB:P06731",
  "gene_name": "Carcinoembryonic antigen-related cell adhesion molecule 5",
  "term_label": "heterophilic cell-cell adhesion",
  "gene_symbol": "CEACAM5",
  "term_id": "GO:0007157"
}